{
  "gene_name": "Toll-like receptor 9",
  "gene": "UniProtKB:Q9NR96",
  "gene_symbol": "TLR9",
  "term_id": "GO:0032755",
  "term_label": "positive regulation of interleukin-6 production"
}